{
  "term_label": "protein targeting to vacuole",
  "term_id": "GO:0006623",
  "gene_symbol": "VPS37D",
  "gene": "UniProtKB:Q86XT2",
  "gene_name": "Vacuolar protein sorting-associated protein 37D"
}